{
  "term_label": "Unknown biological process",
  "gene": "UniProtKB:Q0GE19",
  "gene_symbol": "SLC10A7",
  "term_id": "UNKNOWN:0002",
  "gene_name": "Sodium_bile acid cotransporter 7"
}